microsporocyte differentiation [GO:0010480] (biological process) Definition: The process aimed at the progression of a microsporocyte cell over time, from initial commitment of the cell to a specific fate, to the fully functional differentiated cell. A microsporocyte is a diploid (2n) cell that undergoes meiosis and forms four haploid (1n) microspores; also called microspore mother cell and, in seed plants, pollen mother cell. References: PMID:16751349 Sources: CL:0000248 Also known as: pollen mother cell differentiation Relationships: is a type of GO:0003006; is a type of GO:0048533; is part of anther development [GO:0048653]